sagittal suture morphogenesis [GO:0060367] (biological process) Definition: The process in which the sagittal suture is generated and organized. Sources: GOC:dph, GOC:sl Relationships: is a type of cranial suture morphogenesis [GO:0060363]